aromatic amino acid family biosynthetic process [GO:0009073] (BP) Sources: GOC:go_curators Also known as: aromatic amino acid family anabolism, aromatic amino acid family biosynthesis, aromatic amino acid family formation, aromatic amino acid family synthesis, aromatic amino acid family biosynthetic process, shikimate pathway Definition: The chemical reactions and pathways resulting in the formation of aromatic amino acid family, amino acids with aromatic ring (phenylalanine, tyrosine, tryptophan). Subtypes: L-histidine biosynthetic process [GO:0000105], L-tryptophan biosynthetic process [GO:0000162], 4-aminobenzoate biosynthetic process [GO:0008153], GO:0009095, L-dopa biosynthetic process [GO:1903185] Relationships: is a type of aromatic amino acid metabolic process [GO:0009072]; is a type of GO:0046394